{
  "term_id": "GO:0019202",
  "gene_symbol": "HYKK",
  "gene_name": "Hydroxylysine kinase",
  "term_label": "amino acid kinase activity",
  "gene": "UniProtKB:A2RU49"
}